Golgi transport complex binding [GO:0140164] (molecular function) Definition: Binding to a Golgi transport complex, a multisubunit tethering complex of the CATCHR family. References: PMID:28100664 Sources: GOC:ha Relationships: is a type of GO:0044877 Also known as: COG complex binding